{
  "term_id": "UNKNOWN:0002",
  "term_label": "Unknown biological process",
  "gene_name": "Apoptosis-stimulating of p53 protein 2",
  "gene": "UniProtKB:Q13625",
  "gene_symbol": "TP53BP2"
}